{
  "gene_name": "Protein fuzzy homolog",
  "term_label": "Unknown cellular component",
  "term_id": "UNKNOWN:0003",
  "gene": "UniProtKB:Q9BT04",
  "gene_symbol": "FUZ"
}